{
  "gene_name": "Mastermind-like protein 2",
  "term_id": "GO:0003713",
  "gene_symbol": "MAML2",
  "term_label": "transcription coactivator activity",
  "gene": "UniProtKB:Q8IZL2"
}